{
  "gene_symbol": "FOXC2",
  "term_label": "Unknown cellular component",
  "gene": "UniProtKB:Q99958",
  "gene_name": "Forkhead box protein C2",
  "term_id": "UNKNOWN:0003"
}